{
  "term_label": "actin filament bundle assembly",
  "gene_name": "Protein Shroom1",
  "gene": "UniProtKB:Q2M3G4",
  "term_id": "GO:0051017",
  "gene_symbol": "SHROOM1"
}